{
  "gene": "UniProtKB:Q9BT43",
  "gene_name": "DNA-directed RNA polymerase III subunit RPC7-like",
  "term_label": "Unknown biological process",
  "term_id": "UNKNOWN:0002",
  "gene_symbol": "POLR3GL"
}